{
  "gene_name": "Protein Hook homolog 1",
  "gene_symbol": "HOOK1",
  "term_id": "GO:0030705",
  "gene": "UniProtKB:Q9UJC3",
  "term_label": "cytoskeleton-dependent intracellular transport"
}